{
  "gene_name": "Olfactory receptor 4A47",
  "gene": "UniProtKB:Q6IF82",
  "gene_symbol": "OR4A47",
  "term_id": "GO:0004984",
  "term_label": "olfactory receptor activity"
}